glutamate:sodium symporter activity [GO:0015501] (molecular function) Sources: TC:2.A.27.1.1 Also known as: sodium/excitatory glutamate cotransporter activity, sodium/excitatory glutamate symporter activity Relationships: is a type of amino acid:sodium symporter activity [GO:0005283]; is a type of organic acid:sodium symporter activity [GO:0005343]; is a type of carboxylic acid transmembrane transporter activity [GO:0046943] Definition: Enables the transfer of a solute or solutes from one side of a membrane to the other according to the reaction: glutamate(out) + Na+(out) = glutamate(in) + Na+(in). Subtypes: high-affinity L-glutamate transmembrane transporter activity [GO:0005314]